{
  "term_id": "GO:0008470",
  "gene": "UniProtKB:P26440",
  "gene_symbol": "IVD",
  "gene_name": "Isovaleryl-CoA dehydrogenase, mitochondrial",
  "term_label": "3-methylbutanoyl-CoA dehydrogenase activity"
}